mitotic sister chromatid separation [GO:0051306] (biological process) Relationships: is a type of chromosome separation [GO:0051304]; is_a mitotic cell cycle process [GO:1903047]; is part of mitotic sister chromatid segregation [GO:0000070] Sources: GOC:ai Definition: The process in which sister chromatids are physically detached from each other during mitosis. Also known as: mitotic sister chromatid resolution, sister chromatid separation during mitosis, chromosome separation during mitosis, mitotic chromosome separation Regulation: RO_0002211 by regulation of mitotic sister chromatid separation [GO:0010965]; RO_0002213 by positive regulation of mitotic sister chromatid separation [GO:1901970]; negatively regulated by negative regulation of mitotic sister chromatid separation [GO:2000816]